positive regulation of anthocyanin biosynthetic process [GO:0031542] (biological process) Definition: Any process that activates or increases the frequency, rate or extent of the chemical reactions and pathways resulting in the formation of anthocyanins. Sources: GOC:mah Also known as: positive regulation of anthocyanin anabolism, positive regulation of anthocyanin biosynthesis, positive regulation of anthocyanin formation, positive regulation of anthocyanin synthesis, up regulation of anthocyanin biosynthetic process, up-regulation of anthocyanin biosynthetic process, upregulation of anthocyanin biosynthetic process, activation of anthocyanin biosynthetic process, stimulation of anthocyanin biosynthetic process Relationships: is a type of positive regulation of flavonoid biosynthetic process [GO:0009963]; is a type of positive regulation of anthocyanin metabolic process [GO:0031539]; is a type of regulation of anthocyanin biosynthetic process [GO:0031540]; positively regulates anthocyanin-containing compound biosynthetic process [GO:0009718]